{
  "term_id": "UNKNOWN:0002",
  "gene": "UniProtKB:Q16586",
  "gene_symbol": "SGCA",
  "term_label": "Unknown biological process",
  "gene_name": "Alpha-sarcoglycan"
}